{
  "gene_symbol": "IL17RE",
  "term_label": "interleukin-17 receptor activity",
  "term_id": "GO:0030368",
  "gene": "UniProtKB:Q8NFR9",
  "gene_name": "Interleukin-17 receptor E"
}